regulation of neuron migration [GO:2001222] (biological process) Definition: Any process that modulates the frequency, rate or extent of neuron migration. Sources: GOC:obol Also known as: regulation of neuron chemotaxis, regulation of neuronal migration, regulation of neuron guidance Relationships: is a type of GO:0030334; RO_0002211 neuron migration [GO:0001764] Subtypes: regulation of motor neuron migration [GO:1905483], negative regulation of neuron migration [GO:2001223], GO:2001224